{
  "term_label": "RNA polymerase II general transcription initiation factor activity",
  "term_id": "GO:0016251",
  "gene_name": "Transcription initiation factor TFIID subunit 7",
  "gene": "UniProtKB:Q15545",
  "gene_symbol": "TAF7"
}